{
  "gene_name": "General transcription factor IIF subunit 2",
  "term_id": "GO:0006367",
  "term_label": "transcription initiation at RNA polymerase II promoter",
  "gene": "UniProtKB:P13984",
  "gene_symbol": "GTF2F2"
}